{
  "term_label": "chromatin",
  "gene_symbol": "DSCC1",
  "gene_name": "Sister chromatid cohesion protein DCC1",
  "gene": "UniProtKB:Q9BVC3",
  "term_id": "GO:0000785"
}